{
  "term_label": "Unknown cellular component",
  "term_id": "UNKNOWN:0003",
  "gene": "UniProtKB:Q6ZNX1",
  "gene_symbol": "SHLD3",
  "gene_name": "Shieldin complex subunit 3"
}